positive regulation of lymphocyte chemotaxis [GO:0140131] (biological process) Definition: Any process that activates or increases the frequency, rate or extent of lymphocyte chemotaxis. Subtypes: positive regulation of T cell chemotaxis [GO:0010820], positive regulation of natural killer cell chemotaxis [GO:2000503], positive regulation of B cell chemotaxis [GO:2000538] References: PMID:19255442 Relationships: is a type of positive regulation of leukocyte chemotaxis [GO:0002690]; is a type of GO:1901623; is a type of positive regulation of lymphocyte migration [GO:2000403]; RO_0002213 lymphocyte chemotaxis [GO:0048247]